{
  "gene_symbol": "CHMP2B",
  "term_id": "UNKNOWN:0001",
  "gene_name": "Charged multivesicular body protein 2b",
  "term_label": "Unknown molecular function",
  "gene": "UniProtKB:Q9UQN3"
}